establishment of spindle orientation [GO:0051294] (biological process) Subtypes: GO:0000132, GO:0051296 Definition: Any process that set the alignment of spindle relative to other cellular structures. Relationships: is_a establishment of spindle localization [GO:0051293]; is part of establishment of cell polarity [GO:0030010] Sources: GOC:ai Also known as: orienting of spindle, spindle orientation